cellular response to phorbol 13-acetate 12-myristate [GO:1904628] (biological process) References: PMID:2200903 Sources: GOC:TermGenie, GO_REF:0000071 Also known as: cellular response to TPA, cellular response to phorbol 12-tetradecanoate 13-acetate, cellular response to response to PMA, cellular response to tetradecanoylphorbol acetate Relationships: is_a GO:0071396; is_a cellular response to alcohol [GO:0097306]; is_a GO:1901655; is a type of response to phorbol 13-acetate 12-myristate [GO:1904627] Definition: Any process that results in a change in state or activity of a cell (in terms of movement, secretion, enzyme production, gene expression, etc.) as a result of a phorbol 13-acetate 12-myristate stimulus.